{
  "gene_name": "Dual specificity calcium_calmodulin-dependent 3',5'-cyclic nucleotide phosphodiesterase 1B",
  "gene_symbol": "PDE1B",
  "term_id": "GO:0004117",
  "gene": "UniProtKB:Q01064",
  "term_label": "calmodulin-activated dual specificity 3',5'-cyclic-GMP, 3',5'-cyclic-AMP phosphodiesterase activity"
}